{
  "gene_name": "Troponin I, fast skeletal muscle",
  "term_id": "GO:0060048",
  "term_label": "cardiac muscle contraction",
  "gene_symbol": "TNNI2",
  "gene": "UniProtKB:P48788"
}